{
  "gene_name": "Transmembrane protein 238",
  "term_label": "Unknown biological process",
  "gene_symbol": "TMEM238",
  "gene": "UniProtKB:C9JI98",
  "term_id": "UNKNOWN:0002"
}